{
  "gene": "UniProtKB:O75170",
  "gene_symbol": "PPP6R2",
  "gene_name": "Serine_threonine-protein phosphatase 6 regulatory subunit 2",
  "term_id": "GO:0005634",
  "term_label": "nucleus"
}